{
  "gene_symbol": "ARMC9",
  "term_id": "GO:0005814",
  "gene": "UniProtKB:Q7Z3E5",
  "gene_name": "LisH domain-containing protein ARMC9",
  "term_label": "centriole"
}